{
  "term_id": "GO:0030018",
  "term_label": "Z disc",
  "gene_symbol": "NEXN",
  "gene_name": "Nexilin",
  "gene": "UniProtKB:Q0ZGT2"
}